{
  "gene_symbol": "CASTOR1",
  "term_label": "negative regulation of TORC1 signaling",
  "gene_name": "Cytosolic arginine sensor for mTORC1 subunit 1",
  "term_id": "GO:1904262",
  "gene": "UniProtKB:Q8WTX7"
}